{
  "gene_name": "ADAMTS-like protein 4",
  "gene": "UniProtKB:Q6UY14",
  "gene_symbol": "ADAMTSL4",
  "term_label": "Unknown biological process",
  "term_id": "UNKNOWN:0002"
}